{
  "term_id": "UNKNOWN:0001",
  "term_label": "Unknown molecular function",
  "gene_symbol": "POMZP3",
  "gene": "UniProtKB:Q6PJE2",
  "gene_name": "POM121 and ZP3 fusion protein"
}